pinceau fiber [GO:1990031] (cellular component) Sources: NIF_Subcellular:sao109906988 Definition: Dense plexus formed by the descending collaterals of cerebellar basket cells that wrap around a Purkinje cell axonal initial segment. Relationships: is a type of cellular anatomical structure [GO:0110165]; is part of GO:0030424